{
  "term_id": "GO:0003924",
  "term_label": "GTPase activity",
  "gene_name": "GTP-binding nuclear protein Ran",
  "gene_symbol": "RAN",
  "gene": "UniProtKB:P62826"
}